Latia-luciferin monooxygenase (demethylating) activity [GO:0047098] (molecular function) Sources: EC:1.14.99.21 Relationships: is a type of oxidoreductase activity, acting on paired donors, with incorporation or reduction of molecular oxygen [GO:0016705]; is a type of luciferin monooxygenase activity [GO:0045289] Definition: Catalysis of the reaction: 2 O2 + donor-H2 + Latia luciferin = light + H2O + acceptor + formate + CO2 + oxidized Latia luciferin. Also known as: Latia luciferin monooxygenase (demethylating), Latia-luciferin,hydrogen-donor:oxygen oxidoreductase (demethylating), luciferase (Latia luciferin)